K63-linked deubiquitinase activity [GO:0061578] (molecular function) Relationships: is a type of deubiquitinase activity [GO:0101005] References: PMID:18313383 Sources: GOC:dph, GOC:pg Definition: Hydrolysis of a ubiquitin unit from a ubiquitinated protein linked via the Lys63 residue of ubiquitin. Also known as: K63-specific deubiquitinase activity, Lys63-specific deubiquitinase activity